{
  "gene_symbol": "ATP2C1",
  "term_id": "GO:0005886",
  "gene": "UniProtKB:P98194",
  "gene_name": "Calcium-transporting ATPase type 2C member 1",
  "term_label": "plasma membrane"
}